cellular bud tip polarisome [GO:0031561] (CC) Definition: Protein complex that has a role in determining cell polarity, found at the tip of a growing fungal bud. References: PMID:9632790 Relationships: is_a polarisome [GO:0000133]; is part of cellular bud tip [GO:0005934]